{
  "gene_symbol": "RAB3GAP2",
  "gene_name": "Rab3 GTPase-activating protein non-catalytic subunit",
  "gene": "UniProtKB:Q9H2M9",
  "term_label": "enzyme regulator activity",
  "term_id": "GO:0030234"
}